{
  "gene": "UniProtKB:Q6ICB0",
  "term_label": "protein export from nucleus",
  "term_id": "GO:0006611",
  "gene_name": "Desumoylating isopeptidase 1",
  "gene_symbol": "DESI1"
}